trans-2-decenoyl-acyl-carrier-protein isomerase activity [GO:0034017] (molecular function) Sources: RHEA:23568 Relationships: is a type of intramolecular oxidoreductase activity, transposing C=C bonds [GO:0016863] Definition: Catalysis of the reaction: trans-dec-2-enoyl-[acyl-carrier protein] = cis-dec-3-enoyl-[acyl-carrier protein]. Also known as: beta-hydroxydecanoyl thioester dehydrase activity, trans-2, cis-3 decenoyl-ACP isomerase activity, trans-2, cis-3 decenoyl-[acyl-carrier-protein] isomerase activity, decenoyl-acyl-carrier-protein delta2-trans-delta3-cis-isomerase activity, trans-2,cis-3-decenoyl-ACP isomerase activity, trans-2-cis-3-decenoyl-ACP isomerase activity, trans-2-decenoyl-ACP isomerase activity